intrinsic apoptotic signaling pathway in response to DNA damage [GO:0008630] (biological process) Definition: The series of molecular signals in which an intracellular signal is conveyed to trigger the apoptotic death of a cell. The pathway is induced by the detection of DNA damage, and ends when the execution phase of apoptosis is triggered. Also known as: DNA damage response, signal transduction resulting in induction of apoptosis Sources: GOC:go_curators, GOC:mtg_apoptosis Relationships: is a type of GO:0006974; is a type of intrinsic apoptotic signaling pathway [GO:0097193] Regulation: regulated by regulation of intrinsic apoptotic signaling pathway in response to DNA damage [GO:1902229]; negatively regulated by negative regulation of intrinsic apoptotic signaling pathway in response to DNA damage [GO:1902230]; positively regulated by GO:1902231 Subtypes: intrinsic apoptotic signaling pathway in response to DNA damage by p53 class mediator [GO:0042771]